{
  "gene_symbol": "ZBTB24",
  "gene_name": "Zinc finger and BTB domain-containing protein 24",
  "gene": "UniProtKB:O43167",
  "term_label": "RNA polymerase II cis-regulatory region sequence-specific DNA binding",
  "term_id": "GO:0000978"
}